{
  "gene_symbol": "A0A5F9ZHS0",
  "gene_name": "Uncharacterized protein",
  "term_id": "UNKNOWN:0003",
  "term_label": "Unknown cellular component",
  "gene": "UniProtKB:A0A5F9ZHS0"
}